{
  "gene": "UniProtKB:O43347",
  "gene_symbol": "MSI1",
  "gene_name": "RNA-binding protein Musashi homolog 1",
  "term_label": "regulation of translation",
  "term_id": "GO:0006417"
}